importin-alpha family protein binding [GO:0061676] (molecular function) References: PMID:15350979, PMID:17170104, PMID:23734157 Definition: Binding to a member of the importin-alpha family. Relationships: is a type of GO:0005515